{
  "gene": "UniProtKB:P04114",
  "gene_name": "Apolipoprotein B-100",
  "term_id": "GO:0120020",
  "gene_symbol": "APOB",
  "term_label": "cholesterol transfer activity"
}